{
  "term_label": "extracellular space",
  "gene": "UniProtKB:Q9UK05",
  "gene_symbol": "GDF2",
  "term_id": "GO:0005615",
  "gene_name": "Growth_differentiation factor 2"
}